venom-mediated inhibition of calcium channel activity [GO:0044473] (biological process) Definition: A process in which an organism inhibits or disrupts the activity of a calcium channel in another organism via the action of a venom. References: PMID:20920515 Sources: GOC:fj, GOC:jl Relationships: is_a venom-mediated perturbation of calcium channel activity [GO:0044472] Also known as: envenomation resulting in negative regulation of calcium channel activity in another organism, envenomation resulting in negative regulation of calcium channel activity in other organism Subtypes: venom-mediated inhibition of voltage-gated calcium channel activity [GO:0044474]